{
  "gene": "UniProtKB:P11169",
  "gene_symbol": "SLC2A3",
  "gene_name": "Solute carrier family 2, facilitated glucose transporter member 3",
  "term_id": "GO:0055056",
  "term_label": "D-glucose transmembrane transporter activity"
}